{
  "term_label": "cytoplasm",
  "gene_symbol": "MINK1",
  "term_id": "GO:0005737",
  "gene_name": "Misshapen-like kinase 1",
  "gene": "UniProtKB:Q8N4C8"
}